{
  "gene_name": "Tubulin alpha-1B chain",
  "term_id": "GO:0000226",
  "gene": "UniProtKB:P68363",
  "gene_symbol": "TUBA1B",
  "term_label": "microtubule cytoskeleton organization"
}